exoneme [GO:0044311] (cellular component) Relationships: is a type of intracellular membrane-bounded organelle [GO:0043231]; is part of apical complex [GO:0020007] References: PMID:18083092, PMID:18083098 Sources: GOC:jl Definition: A dense granule-like organelle of the apical complex of merozoites, released into the parasitophorous vacuole, mediating protease-dependent rupture and parasite exit from the infected erythrocyte.